{
  "gene_name": "B melanoma antigen 1",
  "term_id": "UNKNOWN:0003",
  "gene": "UniProtKB:Q13072",
  "term_label": "Unknown cellular component",
  "gene_symbol": "BAGE"
}